{
  "term_label": "type I interferon-mediated signaling pathway",
  "gene_symbol": "STAT2",
  "term_id": "GO:0060337",
  "gene": "UniProtKB:P52630",
  "gene_name": "Signal transducer and activator of transcription 2"
}